{
  "gene_name": "Arylamine N-acetyltransferase 2",
  "gene_symbol": "NAT2",
  "term_id": "UNKNOWN:0002",
  "gene": "UniProtKB:P11245",
  "term_label": "Unknown biological process"
}